{
  "gene": "UniProtKB:Q8WW59",
  "gene_symbol": "SPRYD4",
  "gene_name": "SPRY domain-containing protein 4",
  "term_id": "UNKNOWN:0001",
  "term_label": "Unknown molecular function"
}